{
  "term_id": "GO:0006357",
  "gene_symbol": "KDM2B",
  "gene_name": "Lysine-specific demethylase 2B",
  "term_label": "regulation of transcription by RNA polymerase II",
  "gene": "UniProtKB:Q8NHM5"
}